conidium development [GO:0061794] (biological process) Sources: GOC:di, GOC:dph Relationships: is a type of cell development [GO:0048468] Definition: The process whose specific outcome is the progression of conidium over time, from its formation to the mature structure. Conidia are non-motile spores produced via mitotic asexual reproduction in higher fungi; they are haploid cells genetically identical to their haploid parent. They are produced by conversion of hyphal elements, or are borne on sporogenous cells on or within specialized structures termed conidiophores, and participate in dispersal of the fungus.